{
  "term_label": "G protein-coupled receptor activity",
  "term_id": "GO:0004930",
  "gene": "UniProtKB:O60242",
  "gene_symbol": "ADGRB3",
  "gene_name": "Adhesion G protein-coupled receptor B3"
}